{
  "gene_symbol": "ASPHD1",
  "term_id": "UNKNOWN:0003",
  "term_label": "Unknown cellular component",
  "gene": "UniProtKB:Q5U4P2",
  "gene_name": "Aspartate beta-hydroxylase domain-containing protein 1"
}